{
  "gene_symbol": "RAVER1",
  "term_id": "UNKNOWN:0002",
  "term_label": "Unknown biological process",
  "gene": "UniProtKB:Q8IY67",
  "gene_name": "Ribonucleoprotein PTB-binding 1"
}